{
  "gene": "UniProtKB:Q9Y227",
  "term_label": "UDP phosphatase activity",
  "gene_name": "Ectonucleoside triphosphate diphosphohydrolase 4",
  "gene_symbol": "ENTPD4",
  "term_id": "GO:0045134"
}